nitrite reductase activity [GO:0098809] (molecular function) Relationships: is a type of oxidoreductase activity, acting on other nitrogenous compounds as donors [GO:0016661] Sources: GOC:dos, GOC:jh Subtypes: nitrite reductase [NAD(P)H] activity [GO:0008942], nitrite reductase (cytochrome, ammonia-forming) activity [GO:0042279], GO:0048307, nitrite reductase (NO-forming) activity [GO:0050421] Definition: Catalysis of the reaction: nitrite + acceptor = product(s) of nitrate reduction + reduced acceptor.